{
  "term_label": "Notch signaling pathway",
  "gene_name": "Neurogenic locus notch homolog protein 1",
  "gene": "UniProtKB:P46531",
  "gene_symbol": "NOTCH1",
  "term_id": "GO:0007219"
}